glycerol-3-phosphate dehydrogenase (NADP+) activity [GO:0141153] (molecular function) Relationships: is_a GO:0047952 References: PMID:15557260 Sources: RHEA:11096 Also known as: L-glycerol-3-phosphate:NADP oxidoreductase activity, glycerol phosphate dehydrogenase (nicotinamide adenine dinucleotide phosphate) activity, glycerol-3-phosphate dehydrogenase [NADP+] activity Definition: NADP+ + sn-glycerol 3-phosphate = dihydroxyacetone phosphate + H+ + NADPH.